main axon [GO:0044304] (cellular component) Sources: NIF_Subcellular:sao1596975044 Definition: The main axonal trunk, as opposed to the collaterals; i.e., excluding collaterals, terminal, spines, or dendrites. Also known as: axon trunk, axon shaft, axonal shaft Relationships: is a type of cellular anatomical structure [GO:0110165]; is part of axon [GO:0030424]